{
  "gene": "UniProtKB:Q9Y5H1",
  "gene_name": "Protocadherin gamma-A2",
  "term_id": "GO:0007155",
  "term_label": "cell adhesion",
  "gene_symbol": "PCDHGA2"
}